{
  "term_id": "GO:0015035",
  "gene": "UniProtKB:Q8IXB1",
  "gene_symbol": "DNAJC10",
  "gene_name": "DnaJ homolog subfamily C member 10",
  "term_label": "protein-disulfide reductase activity"
}